{
  "term_id": "UNKNOWN:0002",
  "gene_name": "Urokinase plasminogen activator surface receptor",
  "gene": "UniProtKB:Q03405",
  "gene_symbol": "PLAUR",
  "term_label": "Unknown biological process"
}